{
  "gene_name": "Proline-rich protein 4",
  "term_label": "Unknown biological process",
  "gene_symbol": "PRR4",
  "gene": "UniProtKB:Q16378",
  "term_id": "UNKNOWN:0002"
}